{
  "gene": "UniProtKB:P60331",
  "term_label": "Unknown cellular component",
  "gene_name": "Keratin-associated protein 10-1",
  "gene_symbol": "KRTAP10-1",
  "term_id": "UNKNOWN:0003"
}